adenosine 5'-monophosphoramidase activity [GO:0043530] (molecular function) Definition: Catalysis of the reaction: adenosine 5'-monophosphoramidate + H2O = AMP + NH4+. Other substrates include AMP-morpholidate, AMP-N-alanine methyl ester and AMP-alpha-acetyl lysine methyl ester. References: PMID:11805111 Sources: RHEA:67916 Also known as: adenosine 5' monophosphoramidase activity, adenosine 5'-monophosphoramidate hydrolase activity Relationships: is a type of hydrolase activity, acting on carbon-nitrogen (but not peptide) bonds, in linear amides [GO:0016811]